{
  "term_id": "UNKNOWN:0002",
  "gene_name": "Putative transmembrane protein 217B",
  "gene_symbol": "TMEM217B",
  "gene": "UniProtKB:A0A494BZU4",
  "term_label": "Unknown biological process"
}